{
  "gene": "UniProtKB:P48745",
  "term_label": "integrin binding",
  "gene_name": "CCN family member 3",
  "term_id": "GO:0005178",
  "gene_symbol": "CCN3"
}